{
  "term_id": "GO:0070979",
  "gene": "UniProtKB:Q969T4",
  "term_label": "protein K11-linked ubiquitination",
  "gene_name": "Ubiquitin-conjugating enzyme E2 E3",
  "gene_symbol": "UBE2E3"
}